{
  "gene": "UniProtKB:Q16778",
  "term_id": "GO:0005634",
  "gene_symbol": "H2BC21",
  "gene_name": "Histone H2B type 2-E",
  "term_label": "nucleus"
}